{
  "gene_symbol": "NOS3",
  "gene": "UniProtKB:P29474",
  "term_label": "negative regulation of blood pressure",
  "term_id": "GO:0045776",
  "gene_name": "Nitric oxide synthase 3"
}